{
  "gene_symbol": "TUT4",
  "term_label": "Unknown cellular component",
  "term_id": "UNKNOWN:0003",
  "gene_name": "Terminal uridylyltransferase 4",
  "gene": "UniProtKB:Q5TAX3"
}